{
  "term_label": "Unknown cellular component",
  "gene_symbol": "KCTD4",
  "gene": "UniProtKB:Q8WVF5",
  "gene_name": "BTB_POZ domain-containing protein KCTD4",
  "term_id": "UNKNOWN:0003"
}